{
  "term_id": "GO:0005886",
  "gene_name": "Amphiphysin",
  "gene": "UniProtKB:P49418",
  "gene_symbol": "AMPH",
  "term_label": "plasma membrane"
}